{
  "term_label": "vascular endothelial growth factor receptor 3 binding",
  "gene": "UniProtKB:P49767",
  "term_id": "GO:0043185",
  "gene_name": "Vascular endothelial growth factor C",
  "gene_symbol": "VEGFC"
}